{
  "gene_symbol": "LY6H",
  "term_label": "acetylcholine receptor signaling pathway",
  "gene": "UniProtKB:O94772",
  "gene_name": "Lymphocyte antigen 6H",
  "term_id": "GO:0095500"
}